negative regulation of T cell antigen processing and presentation [GO:0002626] (BP) Definition: Any process that stops, prevents, or reduces the frequency, rate, or extent of T cell antigen processing and presentation. Sources: GOC:add Also known as: down regulation of T cell antigen processing and presentation, down-regulation of T cell antigen processing and presentation, downregulation of T cell antigen processing and presentation, negative regulation of T lymphocyte antigen processing and presentation, negative regulation of T-cell antigen processing and presentation, negative regulation of T-lymphocyte antigen processing and presentation, inhibition of T cell antigen processing and presentation Relationships: is a type of negative regulation of antigen processing and presentation [GO:0002578]; is a type of regulation of T cell antigen processing and presentation [GO:0002625]; is a type of negative regulation of T cell mediated immunity [GO:0002710]; negatively regulates T cell antigen processing and presentation [GO:0002457]